{
  "term_id": "GO:0061136",
  "gene_name": "Proteasome activator complex subunit 1",
  "term_label": "regulation of proteasomal protein catabolic process",
  "gene": "UniProtKB:Q06323",
  "gene_symbol": "PSME1"
}